{
  "term_label": "medium-chain fatty acid catabolic process",
  "gene": "UniProtKB:Q8WU67",
  "term_id": "GO:0051793",
  "gene_symbol": "ABHD3",
  "gene_name": "Phospholipase ABHD3"
}